{
  "gene_symbol": "AMELY",
  "gene": "UniProtKB:Q99218",
  "term_id": "GO:0030345",
  "gene_name": "Amelogenin, Y isoform",
  "term_label": "structural constituent of tooth enamel"
}